16S rRNA (guanine(1207)-N(2))-methyltransferase activity [GO:0052914] (molecular function) Sources: EC:2.1.1.172 Relationships: is a type of rRNA (guanine-N2-)-methyltransferase activity [GO:0008990] Also known as: M(2)G1207 methyltransferase activity Definition: Catalysis of the reaction: S-adenosyl-L-methionine + guanosine(1207) in 16S rRNA = N(2)-methylguanosine(1207) in 16S rRNA + S-adenosyl-L-homocysteine.